{
  "gene_symbol": "PRR27",
  "term_id": "UNKNOWN:0001",
  "gene": "UniProtKB:Q6MZM9",
  "gene_name": "Proline-rich protein 27",
  "term_label": "Unknown molecular function"
}